{
  "gene_symbol": "RPL10L",
  "gene_name": "Ribosomal protein uL16-like",
  "term_label": "male meiosis I",
  "term_id": "GO:0007141",
  "gene": "UniProtKB:Q96L21"
}